negative regulation of substrate-dependent cell migration, cell attachment to substrate [GO:1904236] (BP) Definition: Any process that stops, prevents or reduces the frequency, rate or extent of substrate-dependent cell migration, cell attachment to substrate. Relationships: is a type of negative regulation of cell-substrate adhesion [GO:0010812]; is a type of negative regulation of cell migration [GO:0030336]; is a type of regulation of substrate-dependent cell migration, cell attachment to substrate [GO:1904235]; RO_0002212 substrate-dependent cell migration, cell attachment to substrate [GO:0006931] Also known as: down regulation of substrate-bound cell migration, cell attachment to substrate, down regulation of substrate-dependent cell migration, cell attachment to substrate, down-regulation of substrate-bound cell migration, cell attachment to substrate, down-regulation of substrate-dependent cell migration, cell attachment to substrate, downregulation of substrate-bound cell migration, cell attachment to substrate, downregulation of substrate-dependent cell migration, cell attachment to substrate, negative regulation of substrate-bound cell migration, cell attachment to substrate, inhibition of substrate-bound cell migration, cell attachment to substrate, inhibition of substrate-dependent cell migration, cell attachment to substrate References: PMID:25834989 Sources: GOC:TermGenie, GO_REF:0000058